{
  "term_id": "GO:0003723",
  "gene": "UniProtKB:P41567",
  "gene_symbol": "EIF1",
  "term_label": "RNA binding",
  "gene_name": "Eukaryotic translation initiation factor 1"
}